UDP-xylose transmembrane transport [GO:0015790] (biological process) Relationships: is a type of organic anion transport [GO:0015711]; is a type of pyrimidine nucleotide-sugar transmembrane transport [GO:0090481] Also known as: UDP-xylose transport Sources: GOC:ai Definition: The directed movement of UDP-xylose into, out of or within a cell, or between cells, by means of some agent such as a transporter or pore. UDP-xylose is a substance composed of xylose in glycosidic linkage with uridine diphosphate.